{
  "term_id": "GO:0005769",
  "term_label": "early endosome",
  "gene": "UniProtKB:Q641Q2",
  "gene_symbol": "WASHC2A",
  "gene_name": "WASH complex subunit 2A"
}